{
  "gene_symbol": "PTGS2",
  "term_id": "GO:0004666",
  "gene_name": "Prostaglandin G_H synthase 2",
  "gene": "UniProtKB:P35354",
  "term_label": "prostaglandin-endoperoxide synthase activity"
}